{
  "gene": "UniProtKB:Q9BTE7",
  "gene_name": "DCN1-like protein 5",
  "gene_symbol": "DCUN1D5",
  "term_id": "GO:0045116",
  "term_label": "protein neddylation"
}